regulation of renal amino acid absorption [GO:1902752] (biological process) References: PMID:1526373 Sources: GOC:TermGenie, GOC:hjd, GO_REF:0000058 Relationships: is a type of regulation of renal system process [GO:0098801]; regulates renal amino acid absorption [GO:1990297] Definition: Any process that modulates the frequency, rate or extent of renal amino acid absorption. Subtypes: negative regulation of renal amino acid absorption [GO:1902753], positive regulation of renal amino acid absorption [GO:1902754]